{
  "gene_symbol": "SYT2",
  "gene": "UniProtKB:Q8N9I0",
  "gene_name": "Synaptotagmin-2",
  "term_label": "dense core granule",
  "term_id": "GO:0031045"
}